{
  "gene_symbol": "SNCA",
  "gene": "UniProtKB:P37840",
  "term_label": "cuprous ion binding",
  "gene_name": "Alpha-synuclein",
  "term_id": "GO:1903136"
}